regulation of T-helper 1 cell cytokine production [GO:2000554] (biological process) Sources: GOC:obol Relationships: is a type of GO:0002724; is a type of GO:0002825; regulates T-helper 1 cell cytokine production [GO:0035744] Definition: Any process that modulates the frequency, rate or extent of T-helper 1 cell cytokine production. Subtypes: negative regulation of T-helper 1 cell cytokine production [GO:2000555], positive regulation of T-helper 1 cell cytokine production [GO:2000556] Also known as: regulation of Th1 cell cytokine production